{
  "gene_name": "SEC23-interacting protein",
  "gene": "UniProtKB:Q9Y6Y8",
  "gene_symbol": "SEC23IP",
  "term_label": "cytoplasm",
  "term_id": "GO:0005737"
}